plasma membrane bounded cell projection organization [GO:0120036] (biological process) Sources: GOC:krc Relationships: is a type of cell projection organization [GO:0030030] Subtypes: neuron projection development [GO:0031175], pseudopodium organization [GO:0031268], ruffle organization [GO:0031529], microvillus organization [GO:0032528], GO:0032796, non-sensory hair organization [GO:0035316], GO:0044782, lamellipodium organization [GO:0097581], neuron projection organization [GO:0106027], GO:0120031 Regulation: regulated by regulation of plasma membrane bounded cell projection organization [GO:0120035] Definition: A process that is carried out at the cellular level which results in the assembly, arrangement of constituent parts, or disassembly of a plasma membrane bounded prolongation or process extending from a cell, e.g. a cilium or axon.